{
  "gene": "UniProtKB:P15313",
  "gene_name": "V-type proton ATPase subunit B, kidney isoform",
  "gene_symbol": "ATP6V1B1",
  "term_id": "UNKNOWN:0001",
  "term_label": "Unknown molecular function"
}